histone methacryltransferase activity [GO:0140218] (MF) Also known as: histone 2-methylpropenoyl transferase activity Relationships: is a type of histone modifying activity [GO:0140993] Definition: Catalysis of the reaction: 2-methylpropenoyl-CoA + L-lysyl-[protein] = N6-methacrylyl-L-lysyl-[protein] + CoA + H+. Methacryl-CoA is a synonym of 2-methylpropenoyl-CoA. References: PMID:34961760, PMID:40339582